{
  "term_id": "UNKNOWN:0003",
  "gene_symbol": "EIF4EBP3",
  "gene_name": "Eukaryotic translation initiation factor 4E-binding protein 3",
  "term_label": "Unknown cellular component",
  "gene": "UniProtKB:O60516"
}